negative regulation of receptor catabolic process [GO:2000645] (biological process) Subtypes: negative regulation of low-density lipoprotein particle receptor catabolic process [GO:0032804] Sources: GOC:BHF Also known as: negative regulation of receptor breakdown, negative regulation of receptor catabolism, negative regulation of receptor degradation Definition: Any process that stops, prevents or reduces the frequency, rate or extent of receptor catabolic process. Relationships: is a type of GO:0009895; is a type of negative regulation of macromolecule metabolic process [GO:0010605]; is a type of regulation of receptor catabolic process [GO:2000644]; negatively regulates receptor catabolic process [GO:0032801]